{
  "term_label": "nucleus",
  "gene_name": "Histone H2A.J",
  "gene": "UniProtKB:Q9BTM1",
  "gene_symbol": "H2AJ",
  "term_id": "GO:0005634"
}